glycochenodeoxycholate sulfotransferase activity [GO:0033876] (molecular function) Relationships: is a type of GO:0008146 Sources: EC:2.8.2.34, RHEA:17689 Also known as: bile acid:3'-phosphoadenosine-5'-phosphosulfate sulfotransferase activity, 3'-phosphoadenylyl-sulfate:glycochenodeoxycholate 7-sulfotransferase activity, BAST, bile acid:PAPS:sulfotransferase activity Definition: Catalysis of the reaction: 3'-phospho-5'-adenylyl sulfate + glycochenodeoxycholate = adenosine 3',5'-diphosphate + glycochenodeoxycholate 7-sulfate + H+.